{
  "term_id": "GO:0016581",
  "term_label": "NuRD complex",
  "gene_name": "Chromodomain-helicase-DNA-binding protein 4",
  "gene": "UniProtKB:Q14839",
  "gene_symbol": "CHD4"
}